{
  "gene_symbol": "SLC5A7",
  "term_label": "synaptic transmission, cholinergic",
  "term_id": "GO:0007271",
  "gene": "UniProtKB:Q9GZV3",
  "gene_name": "High affinity choline transporter 1"
}